{
  "term_id": "GO:0005634",
  "gene": "UniProtKB:O15055",
  "gene_symbol": "PER2",
  "term_label": "nucleus",
  "gene_name": "Period circadian protein homolog 2"
}